DNA biosynthetic process [GO:0071897] (biological process) Definition: The biosynthetic process resulting in the formation of DNA. Sources: GOC:mah Also known as: DNA anabolism, DNA biosynthesis, DNA formation, DNA synthesis Relationships: is a type of DNA metabolic process [GO:0006259]; is a type of nucleic acid biosynthetic process [GO:0141187] Subtypes: DNA synthesis involved in DNA repair [GO:0000731], DNA amplification [GO:0006277], RNA-templated DNA biosynthetic process [GO:0006278], viral DNA genome replication [GO:0039693], DNA synthesis involved in DNA replication [GO:0090592] Regulation: regulated by GO:2000278; negatively regulated by negative regulation of DNA biosynthetic process [GO:2000279]; positively regulated by positive regulation of DNA biosynthetic process [GO:2000573]